positive regulation of MDA-5 signaling pathway [GO:1900245] (biological process) Sources: GOC:TermGenie Relationships: is a type of positive regulation of immune effector process [GO:0002699]; is a type of regulation of MDA-5 signaling pathway [GO:0039533]; is a type of positive regulation of pattern recognition receptor signaling pathway [GO:0062208]; is a type of positive regulation of intracellular signal transduction [GO:1902533]; positively regulates MDA-5 signaling pathway [GO:0039530] Also known as: positive regulation of IFIH1 signaling pathway, positive regulation of MDA-5 signalling pathway, positive regulation of melanoma differentiation-associated gene 5 signaling pathway, up regulation of IFIH1 signaling pathway, up regulation of MDA-5 signaling pathway, up regulation of melanoma differentiation-associated gene 5 signaling pathway, up-regulation of IFIH1 signaling pathway, up-regulation of MDA-5 signaling pathway, up-regulation of melanoma differentiation-associated gene 5 signaling pathway, upregulation of IFIH1 signaling pathway, upregulation of MDA-5 signaling pathway, upregulation of melanoma differentiation-associated gene 5 signaling pathway, activation of IFIH1 signaling pathway, activation of MDA-5 signaling pathway, activation of MDA5 signaling pathway, activation of melanoma differentiation-associated gene 5 signaling pathway, positive regulation of MDA5 signaling pathway, up regulation of MDA5 signaling pathway, up-regulation of MDA5 signaling pathway, upregulation of MDA5 signaling pathway Definition: Any process that activates or increases the frequency, rate or extent of MDA-5 signaling pathway.